molybdopterin cofactor binding [GO:0043546] (MF) Relationships: is a type of binding [GO:0005488] Also known as: Moco binding Definition: Binding to a molybdopterin cofactor (Moco), essential for the catalytic activity of some enzymes, e.g. sulfite oxidase, xanthine dehydrogenase, and aldehyde oxidase. The cofactor consists of a mononuclear molybdenum (Mo-molybdopterin) or tungsten ion (W-molybdopterin) coordinated by one or two molybdopterin ligands. Sources: ISSN:09498257